mitochondrial translation initiation complex [GO:0180052] (cellular component) Also known as: mtIC, mitochondrial initiation complex References: PMID:32522994 Sources: GOC:vw Definition: A ribonucleoprotein complex comprising the mRNA bound fully assembled 55S mitoribosome with the tRNA-met positioned in the P-site of the mitochondrial small subunit to recognize the mRNA start codon. Relationships: is_a translation initiation complex [GO:0070992]; is a type of mitochondrial protein-containing complex [GO:0098798]; is part of mitochondrial matrix [GO:0005759]